{
  "gene_symbol": "SPTLC3",
  "gene": "UniProtKB:Q9NUV7",
  "term_label": "serine C-palmitoyltransferase activity",
  "gene_name": "Serine palmitoyltransferase 3",
  "term_id": "GO:0004758"
}